{
  "gene": "UniProtKB:Q8IZD9",
  "term_id": "GO:0005085",
  "gene_symbol": "DOCK3",
  "term_label": "guanyl-nucleotide exchange factor activity",
  "gene_name": "Dedicator of cytokinesis protein 3"
}